{
  "term_label": "Unknown biological process",
  "gene_name": "Putative uncharacterized protein encoded by LINC02910",
  "gene": "UniProtKB:Q8N268",
  "gene_symbol": "LINC02910",
  "term_id": "UNKNOWN:0002"
}